{
  "term_id": "GO:0006357",
  "term_label": "regulation of transcription by RNA polymerase II",
  "gene_name": "ETS-related transcription factor Elf-3",
  "gene_symbol": "ELF3",
  "gene": "UniProtKB:P78545"
}